negative regulation of keratinocyte proliferation [GO:0010839] (BP) Definition: Any process that decreases the rate, frequency or extent of keratinocyte proliferation. Keratinocyte proliferation is the multiplication or reproduction of keratinocytes, resulting in the expansion of a cell population. Sources: GOC:dph, GOC:tb Relationships: is a type of regulation of keratinocyte proliferation [GO:0010837]; is a type of negative regulation of epithelial cell proliferation [GO:0050680]; negatively regulates GO:0043616